{
  "gene": "UniProtKB:O43924",
  "gene_name": "Retinal rod rhodopsin-sensitive cGMP 3',5'-cyclic phosphodiesterase subunit delta",
  "gene_symbol": "PDE6D",
  "term_label": "Unknown molecular function",
  "term_id": "UNKNOWN:0001"
}